cellular response to X-ray [GO:0071481] (BP) Also known as: cellular response to X-ray radiation stimulus Definition: Any process that results in a change in state or activity of a cell (in terms of movement, secretion, enzyme production, gene expression, etc.) as a result of X-ray radiation. An X-ray is a form of electromagnetic radiation with a wavelength in the range of 10 nanometers to 100 picometers (corresponding to frequencies in the range 30 PHz to 3 EHz). Relationships: is a type of response to X-ray [GO:0010165]; is_a GO:0071479 Sources: GOC:mah Regulation: regulated by GO:2000683; negatively regulated by GO:2000684; positively regulated by positive regulation of cellular response to X-ray [GO:2000685]